ventral spinal cord interneuron fate commitment [GO:0060579] (biological process) Definition: The process in which the developmental fate of a cell becomes restricted such that it will develop into a ventral spinal cord interneuron. Ventral spinal cord interneurons are cells located in the ventral portion of the spinal cord that transmit signals between sensory and motor neurons and are required for reflexive responses. Sources: GOC:dph Relationships: is a type of neuron fate commitment [GO:0048663]; is a type of cell fate commitment involved in pattern specification [GO:0060581]; is part of spinal cord dorsal/ventral patterning [GO:0021513]; is part of ventral spinal cord interneuron differentiation [GO:0021514]